{
  "gene_name": "DNA dC-dU-editing enzyme APOBEC-3C",
  "term_label": "DNA cytosine deamination",
  "term_id": "GO:0070383",
  "gene_symbol": "APOBEC3C",
  "gene": "UniProtKB:Q9NRW3"
}